cellular response to hypoxia [GO:0071456] (biological process) Regulation: regulated by GO:1900037; negatively regulated by negative regulation of cellular response to hypoxia [GO:1900038]; positively regulated by GO:1900039 Also known as: cellular response to hypoxic stress, cellular response to lowered oxygen tension Definition: Any process that results in a change in state or activity of a cell (in terms of movement, secretion, enzyme production, gene expression, etc.) as a result of a stimulus indicating lowered oxygen tension. Hypoxia, defined as a decline in O2 levels below normoxic levels of 20.8 - 20.95%, results in metabolic adaptation at both the cellular and organismal level. Relationships: is a type of GO:0001666; is_a GO:0033554; is_a cellular response to decreased oxygen levels [GO:0036294] Note: Note that this term should not be confused with 'cellular response to anoxia ; GO:0071454'. Note that in laboratory studies, hypoxia is typically studied at O2 concentrations ranging from 0.1 - 5%. Sources: GOC:mah